FMN hydrolase activity [GO:0090711] (molecular function) Relationships: is a type of phosphatase activity [GO:0016791] Also known as: FMN phosphatase References: PMID:16183635 Sources: RHEA:35587 Definition: Catalysis of the reaction: FMN + H2O = phosphate + riboflavin.